{
  "gene_name": "Double homeobox protein 5",
  "gene": "UniProtKB:Q96PT3",
  "gene_symbol": "DUX5",
  "term_id": "GO:0005634",
  "term_label": "nucleus"
}